{
  "gene": "UniProtKB:P09110",
  "gene_name": "3-ketoacyl-CoA thiolase, peroxisomal",
  "term_label": "acetyl-CoA C-acyltransferase activity",
  "term_id": "GO:0003988",
  "gene_symbol": "ACAA1"
}